perinuclear region of cytoplasm [GO:0048471] (cellular component) Relationships: is a type of cellular anatomical structure [GO:0110165]; is part of GO:0005737 Subtypes: cytoplasmic periphery of the nuclear pore complex [GO:1990723] Note: Note that this term should not be confused with the cellular component term 'nuclear membrane lumen ; GO:0005641', which has the synonym 'perinuclear space'. Definition: Cytoplasm situated near, or occurring around, the nucleus. Sources: GOC:jid